{
  "term_label": "Unknown molecular function",
  "gene_symbol": "CUZD1",
  "gene": "UniProtKB:Q86UP6",
  "term_id": "UNKNOWN:0001",
  "gene_name": "CUB and zona pellucida-like domain-containing protein 1"
}